{
  "term_label": "plasma membrane",
  "gene": "UniProtKB:Q96HU8",
  "gene_symbol": "DIRAS2",
  "gene_name": "GTP-binding protein Di-Ras2",
  "term_id": "GO:0005886"
}